SREBP-SCAP complex [GO:0032936] (cellular component) References: PMID:12923525 Definition: A protein complex formed by the association of sterol regulatory element binding protein (SREBP) and SREBP-cleavage-activating protein (SCAP) in the ER membrane; in the absence of sterols, the SREBP-SCAP complex is packaged into COPII vesicles and travels to the Golgi apparatus to be processed. Relationships: is_a membrane protein complex [GO:0098796] Also known as: Sre1-Scp1 complex